{
  "gene_name": "Serine protease HTRA3",
  "term_label": "Unknown cellular component",
  "gene_symbol": "HTRA3",
  "gene": "UniProtKB:P83110",
  "term_id": "UNKNOWN:0003"
}